{
  "term_label": "P-body assembly",
  "gene_name": "Enhancer of mRNA-decapping protein 3",
  "term_id": "GO:0033962",
  "gene_symbol": "EDC3",
  "gene": "UniProtKB:Q96F86"
}